mesonephric comma-shaped body morphogenesis [GO:0061236] (biological process) Definition: The process in which the mesonephric comma-shaped body is generated and organized. The mesonephric comma-shaped body is the precursor structure to the mesonephric S-shaped body that contributes to the morphogenesis of a nephron in the mesonephros. Relationships: is a type of comma-shaped body morphogenesis [GO:0072049]; is part of GO:0061228 Sources: GOC:mtg_kidney_jan10